formate dehydrogenase (coenzyme F420) activity [GO:0043794] (molecular function) Definition: Catalysis of the reaction: formate + 2 H+ + oxidized coenzyme F420-(gamma-L-Glu)(n) = CO2 + reduced coenzyme F420-(gamma-L-Glu)(n). Also known as: formate dehydrogenase (F420) activity References: PMID:3801411 Sources: RHEA:42764 Relationships: is a type of oxidoreductase activity, acting on CH or CH2 groups [GO:0016725]